heterocyclic compound binding [GO:1901363] (molecular function) Definition: Binding to heterocyclic compound. Subtypes: nucleotide binding [GO:0000166], nucleoside binding [GO:0001882], GO:0002054, folic acid binding [GO:0005542], vitamin E binding [GO:0008431], penicillin binding [GO:0008658], GO:0009374, cocaine binding [GO:0019811], thiamine binding [GO:0030975], thiamine pyrophosphate binding [GO:0030976], lipoic acid binding [GO:0031405], L-ascorbic acid binding [GO:0031418], cobalamin binding [GO:0031419], ectoine binding [GO:0033294], hydroxyectoine binding [GO:0033295], GO:0035639, serotonin binding [GO:0051378], GO:0051381, GO:0051870, dihydrofolic acid binding [GO:0051871], vitamin B6 binding [GO:0070279], GO:0070967, pyrroloquinoline quinone binding [GO:0070968], ADP-D-ribose binding [GO:0072570], flavanol binding [GO:0097245], coenzyme A binding [GO:0120225], acyl-CoA binding [GO:0120227], tryptophan binding [GO:0120284], dethiobiotin binding [GO:1901602], GO:1901707, proline binding [GO:1901973], riboflavin binding [GO:1902444], enterobactin binding [GO:1903981] Relationships: is a type of small molecule binding [GO:0036094] Sources: GOC:TermGenie